{
  "gene_name": "Putative uncharacterized protein FLJ33307",
  "term_label": "Unknown biological process",
  "gene_symbol": "Q8NBF4",
  "term_id": "UNKNOWN:0002",
  "gene": "UniProtKB:Q8NBF4"
}